synaptobrevin 2-SNAP-25-syntaxin-4 complex [GO:0070047] (cellular component) Definition: A SNARE complex that contains synaptobrevin 2 (VAMP2), SNAP-25, and syntaxin 4 (or orthologs thereof). References: PMID:10336434 Also known as: SNARE complex (Stx4, Snap25, Vamp2), Stx4-Snap25-Vamp2 complex Relationships: is a type of SNARE complex [GO:0031201]